{
  "gene": "UniProtKB:Q9BUN8",
  "term_id": "GO:0005047",
  "gene_name": "Derlin-1",
  "gene_symbol": "DERL1",
  "term_label": "signal recognition particle binding"
}